phosphoglycerate transmembrane transporter activity [GO:0015120] (molecular function) Relationships: is a type of aldonate transmembrane transporter activity [GO:0042879]; is part of phosphoglycerate transmembrane transport [GO:0015713] Definition: Enables the transfer of phosphoglycerates from one side of a membrane to the other. Phosphoglycerates are important intermediates in glycolysis and 3-phosphoglycerate is a precursor in serine biosynthesis. Sources: GOC:ai